{
  "gene_symbol": "ZDHHC19",
  "gene": "UniProtKB:Q8WVZ1",
  "term_id": "GO:0005794",
  "gene_name": "Palmitoyltransferase ZDHHC19",
  "term_label": "Golgi apparatus"
}